bundle of His cell to Purkinje myocyte signaling [GO:0086028] (BP) Relationships: is a type of cell-cell signaling involved in cardiac conduction [GO:0086019]; is a type of bundle of His cell to Purkinje myocyte communication [GO:0086069] Also known as: bundle of His cardiac muscle cell to Purkinje myocyte signaling, bundle of His cardiac muscle cell to Purkinje myocyte signalling Sources: GOC:BHF, GOC:mtg_cardiac_conduct_nov11 Definition: Any process that mediates the transfer of information from a bundle of His cardiomyocyte to a Purkinje myocyte.